regulation of heart looping [GO:1901207] (biological process) Sources: GOC:BHF, GOC:TermGenie Also known as: regulation of cardiac looping Definition: Any process that modulates the frequency, rate or extent of heart looping. Relationships: is a type of regulation of morphogenesis of an epithelium [GO:1905330]; regulates GO:0001947 Subtypes: GO:1901208, positive regulation of heart looping [GO:1901209]